{
  "gene_name": "Ecto-ADP-ribosyltransferase 4",
  "term_label": "Unknown cellular component",
  "term_id": "UNKNOWN:0003",
  "gene": "UniProtKB:Q93070",
  "gene_symbol": "ART4"
}